{
  "term_label": "sperm axoneme assembly",
  "gene_name": "Armadillo repeat-containing protein 2",
  "gene": "UniProtKB:Q8NEN0",
  "gene_symbol": "ARMC2",
  "term_id": "GO:0007288"
}